threonine-type peptidase activity [GO:0070003] (molecular function) Sources: GOC:mah, https://www.ebi.ac.uk/merops/about/glossary.shtml#CATTYPE Definition: Catalysis of the hydrolysis of peptide bonds in a polypeptide chain by a mechanism in which the hydroxyl group of a threonine residue at the active center acts as a nucleophile. Relationships: is a type of GO:0008233 Subtypes: GO:0004298, beta-aspartyl-peptidase activity [GO:0008798], glutathione hydrolase activity [GO:0036374]